{
  "term_id": "GO:0003735",
  "gene": "UniProtKB:P0CG47",
  "gene_symbol": "UBB",
  "term_label": "structural constituent of ribosome",
  "gene_name": "Polyubiquitin-B"
}